negative regulation of endosomal vesicle fusion [GO:1905362] (biological process) Also known as: down regulation of endosomal vesicle fusion, down regulation of endosome vesicle fusion, down-regulation of endosomal vesicle fusion, down-regulation of endosome vesicle fusion, downregulation of endosomal vesicle fusion, downregulation of endosome vesicle fusion, negative regulation of endosome vesicle fusion, inhibition of endosomal vesicle fusion, inhibition of endosome vesicle fusion Relationships: is a type of GO:0031339; is a type of regulation of endosomal vesicle fusion [GO:1905364]; negatively regulates endosomal vesicle fusion [GO:0034058] References: PMID:26911690 Sources: GOC:PARL, GOC:TermGenie, GOC:bc, GO_REF:0000058 Definition: Any process that stops, prevents or reduces the frequency, rate or extent of endosomal vesicle fusion.